{
  "gene_symbol": "TNIK",
  "gene_name": "TRAF2 and NCK-interacting protein kinase",
  "term_id": "GO:0004674",
  "term_label": "protein serine/threonine kinase activity",
  "gene": "UniProtKB:Q9UKE5"
}